{
  "gene": "UniProtKB:P07919",
  "term_label": "Unknown molecular function",
  "gene_symbol": "UQCRH",
  "gene_name": "Cytochrome b-c1 complex subunit 6, mitochondrial",
  "term_id": "UNKNOWN:0001"
}